{
  "gene": "UniProtKB:Q8NH05",
  "gene_symbol": "OR4Q3",
  "gene_name": "Olfactory receptor 4Q3",
  "term_label": "Unknown biological process",
  "term_id": "UNKNOWN:0002"
}